{
  "gene": "UniProtKB:Q9UK32",
  "term_label": "nucleoplasm",
  "gene_name": "Ribosomal protein S6 kinase alpha-6",
  "term_id": "GO:0005654",
  "gene_symbol": "RPS6KA6"
}